dihydrosphingosine-1-P pathway [GO:0006648] (biological process) References: PMID:15643073 Sources: GOC:mah Relationships: is a type of phosphatidylethanolamine biosynthetic process [GO:0006646] Definition: A phosphatidylethanolamine biosynthetic process that proceeds via the enzymatic action of dihydrosphingosine phosphate lyase.